{
  "gene_name": "YTH domain-containing family protein 2",
  "term_id": "GO:0061157",
  "term_label": "mRNA destabilization",
  "gene": "UniProtKB:Q9Y5A9",
  "gene_symbol": "YTHDF2"
}